regulation of fear response [GO:1903365] (biological process) Subtypes: negative regulation of fear response [GO:1903366], positive regulation of fear response [GO:1903367], GO:2000822 Definition: Any process that modulates the frequency, rate or extent of fear response. References: PMID:8677262 Sources: GOC:TermGenie, GOC:mr, GO_REF:0000058 Also known as: regulation of physiological fear response Relationships: is a type of regulation of multicellular organismal process [GO:0051239]; is_a regulation of response to stress [GO:0080134]; regulates fear response [GO:0042596]